{
  "term_id": "GO:0006511",
  "term_label": "ubiquitin-dependent protein catabolic process",
  "gene_name": "E3 ubiquitin-protein ligase RBX1",
  "gene_symbol": "RBX1",
  "gene": "UniProtKB:P62877"
}